{
  "gene_name": "Connector enhancer of kinase suppressor of ras 2",
  "term_label": "glutamatergic synapse",
  "gene_symbol": "CNKSR2",
  "gene": "UniProtKB:Q8WXI2",
  "term_id": "GO:0098978"
}